{
  "gene_symbol": "SLC51B",
  "term_label": "basolateral plasma membrane",
  "gene": "UniProtKB:Q86UW2",
  "term_id": "GO:0016323",
  "gene_name": "Organic solute transporter subunit beta"
}